{
  "gene_name": "Golgin subfamily A member 6-like protein 10",
  "term_id": "UNKNOWN:0002",
  "term_label": "Unknown biological process",
  "gene": "UniProtKB:A6NI86",
  "gene_symbol": "GOLGA6L10"
}